{
  "gene_symbol": "GPR21",
  "gene": "UniProtKB:Q99679",
  "gene_name": "Probable G-protein coupled receptor 21",
  "term_id": "GO:0007186",
  "term_label": "G protein-coupled receptor signaling pathway"
}